negative regulation of calcium import into the mitochondrion [GO:0110099] (biological process) Definition: Any process that stops, prevents or reduces the frequency, rate or extent of calcium ion import into the mitochondrion. References: PMID:24085037 Sources: GOC:sl Relationships: is a type of GO:0110097; is_a negative regulation of calcium ion transmembrane transport [GO:1903170]; negatively regulates calcium import into the mitochondrion [GO:0036444]